{
  "gene_name": "Zinc-regulated GTPase metalloprotein activator 1B",
  "term_label": "zinc ion binding",
  "gene": "UniProtKB:Q8IUF1",
  "term_id": "GO:0008270",
  "gene_symbol": "ZNG1B"
}